{
  "gene_name": "Bone morphogenetic protein 6",
  "gene_symbol": "BMP6",
  "gene": "UniProtKB:P22004",
  "term_id": "GO:0030509",
  "term_label": "BMP signaling pathway"
}